metanephric long nephron development [GO:0072238] (biological process) Definition: The process whose specific outcome is the progression of a metanephric long nephron over time, from its formation to the mature structure. Long nephrons are associated with juxtamedullary glomeruli and extend into the inner medulla in the metanephros. Also known as: metanephric juxtamedullary nephron development Relationships: is a type of long nephron development [GO:0072029]; is a type of GO:0072210 Sources: GOC:mtg_kidney_jan10